site-specific telomere resolvase activity [GO:0043336] (molecular function) Note: Note that while this enzyme uses a similar reaction chemistry to topoisomerases and site-specific recombinases, it performs a unique reaction. Topoisomerases promote breakage and reunion of either one or two DNA strands to alter the topological state of a DNA molecule. Site-specific recombinases perform a more complex reaction in which four strands are broken and subsequently joined to a different DNA duplex, resulting in the production of a recombinant product. The telomere resolvases on the other hand, must break two phosphodiester bonds in a single DNA duplex (one on each strand) and join each end with the opposite DNA strand to form covalently closed hairpin telomeres. Definition: Catalysis of a site-specific breakage and reunion reaction that generates two hairpin telomeres from a replicated telomere substrate. Occurs via a two-step transesterification with a protein-DNA intermediate similar to that used by topoisomerases and site-specific recombinases. References: PMID:11804598 Sources: GOC:jl Relationships: is a type of catalytic activity, acting on DNA [GO:0140097]; is part of GO:0000723 Also known as: ResT, TelN